{
  "gene_symbol": "CEP126",
  "gene": "UniProtKB:Q9P2H0",
  "term_label": "cilium assembly",
  "gene_name": "Centrosomal protein of 126 kDa",
  "term_id": "GO:0060271"
}